{
  "term_label": "cellular response to L-leucine",
  "gene_symbol": "SESN3",
  "gene_name": "Sestrin-3",
  "term_id": "GO:0071233",
  "gene": "UniProtKB:P58005"
}